{
  "gene": "UniProtKB:A0A075B6Y4",
  "gene_symbol": "TRAJ19",
  "term_label": "Unknown biological process",
  "term_id": "UNKNOWN:0002",
  "gene_name": "T cell receptor alpha joining 19 (non-functional) (Fragment)"
}